{
  "gene": "UniProtKB:P25054",
  "term_id": "GO:0008017",
  "gene_name": "Adenomatous polyposis coli protein",
  "gene_symbol": "APC",
  "term_label": "microtubule binding"
}